{
  "term_label": "nucleus",
  "term_id": "GO:0005634",
  "gene_symbol": "ZNF585A",
  "gene_name": "Zinc finger protein 585A",
  "gene": "UniProtKB:Q6P3V2"
}